{
  "term_label": "growth factor activity",
  "term_id": "GO:0008083",
  "gene": "UniProtKB:O15520",
  "gene_symbol": "FGF10",
  "gene_name": "Fibroblast growth factor 10"
}